{
  "gene_name": "Chondroadherin-like protein",
  "gene": "UniProtKB:Q6NUI6",
  "term_label": "extracellular matrix",
  "term_id": "GO:0031012",
  "gene_symbol": "CHADL"
}